{
  "gene": "UniProtKB:Q5HY64",
  "term_id": "UNKNOWN:0003",
  "term_label": "Unknown cellular component",
  "gene_name": "Putative protein FAM47C",
  "gene_symbol": "FAM47C"
}